cellular response to differentiation-inducing factor 1 [GO:1903014] (biological process) Definition: Any process that results in a change in state or activity of a cell (in terms of movement, secretion, enzyme production, gene expression, etc.) as a result of a 1-(3,5-dichloro-2,6-dihydroxy-4-methoxyphenyl)hexan-1-one stimulus. References: PMID:22365144 Sources: GOC:TermGenie, GO_REF:0000071 Also known as: cellular response to 1-(3,5-dichloro-2,6-dihydroxy-4-methoxyphenyl)hexan-1-one, DIF-1, cellular response to DIF-1, cellular response to DIF1 Relationships: is a type of cellular response to ether [GO:0071362]; is a type of GO:1901655; is a type of response to differentiation-inducing factor 1 [GO:1903013]